host cell mitochondrial outer membrane [GO:0044193] (cellular component) Relationships: is a type of host organelle outer membrane [GO:0039661]; is a type of GO:0044191 Definition: The outer, i.e. cytoplasm-facing, lipid bilayer of the host cell mitochondrial envelope. Sources: GOC:jl